histamine secretion involved in inflammatory response [GO:0002441] (biological process) Definition: The regulated release of histamine by a cell as part of an inflammatory response. Subtypes: GO:0002553, GO:0002555, histamine secretion by basophil [GO:0002557], GO:0097280 Sources: GOC:add, ISBN:0781735149 Relationships: is a type of histamine secretion [GO:0001821]; is a type of GO:0046879; is part of GO:0002349 Also known as: histamine secretion involved in acute inflammatory response